{
  "term_id": "GO:0004930",
  "term_label": "G protein-coupled receptor activity",
  "gene": "UniProtKB:Q86SQ4",
  "gene_symbol": "ADGRG6",
  "gene_name": "Adhesion G-protein coupled receptor G6"
}